{
  "term_id": "UNKNOWN:0002",
  "term_label": "Unknown biological process",
  "gene_symbol": "THAP3",
  "gene_name": "THAP domain-containing protein 3",
  "gene": "UniProtKB:Q8WTV1"
}